{
  "term_id": "UNKNOWN:0002",
  "gene": "UniProtKB:O75822",
  "gene_symbol": "EIF3J",
  "gene_name": "Eukaryotic translation initiation factor 3 subunit J",
  "term_label": "Unknown biological process"
}